{
  "term_label": "Unknown cellular component",
  "gene_name": "Beta-crystallin A2",
  "gene": "UniProtKB:P53672",
  "gene_symbol": "CRYBA2",
  "term_id": "UNKNOWN:0003"
}